6-aminohexanoate-cyclic-dimer hydrolase activity [GO:0019874] (molecular function) Definition: Catalysis of the reaction: 1,8-diazacyclotetradecane-2,9-dione + H2O = N-(6-aminohexanoyl)-6-aminohexanoate. Also known as: 1,8-diazacyclotetradecane-2,9-dione lactamhydrolase activity Relationships: is_a hydrolase activity, acting on carbon-nitrogen (but not peptide) bonds, in cyclic amides [GO:0016812] Sources: EC:3.5.2.12, RHEA:16225